L-ornithine catabolic process [GO:0006593] (biological process) Sources: GOC:jl, ISBN:0192801023 Also known as: ornithine breakdown, ornithine catabolism, ornithine degradation Subtypes: GO:0019466, L-ornithine catabolic process, by decarboxylation [GO:0019467] Relationships: is a type of ornithine metabolic process [GO:0006591]; is_a L-amino acid catabolic process [GO:0170035]; is a type of GO:0170044 Definition: The chemical reactions and pathways resulting in the breakdown of L-ornithine, an amino acid only rarely found in proteins, but which is important in living organisms as an intermediate in the reactions of the urea cycle and in arginine biosynthesis. Regulation: regulated by GO:1903266; negatively regulated by negative regulation of ornithine catabolic process [GO:1903267]; positively regulated by GO:1903268